{
  "gene_symbol": "BNIP2",
  "gene_name": "BCL2_adenovirus E1B 19 kDa protein-interacting protein 2",
  "gene": "UniProtKB:Q12982",
  "term_id": "UNKNOWN:0001",
  "term_label": "Unknown molecular function"
}